establishment or maintenance of microtubule cytoskeleton polarity [GO:0030951] (biological process) Definition: Any cellular process that results in the specification, formation or maintenance of polarized microtubule-based cytoskeletal structures. Relationships: is a type of microtubule cytoskeleton organization [GO:0000226]; is a type of establishment or maintenance of cytoskeleton polarity [GO:0030952] Subtypes: oocyte microtubule cytoskeleton organization [GO:0016325] Sources: GOC:mah